{
  "gene_name": "Homeobox protein aristaless-like 4",
  "gene": "UniProtKB:Q9H161",
  "term_label": "neuron development",
  "term_id": "GO:0048666",
  "gene_symbol": "ALX4"
}